{
  "gene": "UniProtKB:Q3LHN0",
  "gene_name": "Keratin-associated protein 25-1",
  "term_label": "Unknown molecular function",
  "gene_symbol": "KRTAP25-1",
  "term_id": "UNKNOWN:0001"
}